{
  "gene_name": "Cytoplasmic FMR1-interacting protein 1",
  "term_id": "GO:0000902",
  "term_label": "cell morphogenesis",
  "gene_symbol": "CYFIP1",
  "gene": "UniProtKB:Q7L576"
}